{
  "gene_symbol": "CHN1",
  "gene_name": "N-chimaerin",
  "term_label": "GTPase activator activity",
  "term_id": "GO:0005096",
  "gene": "UniProtKB:P15882"
}